citrate synthase activity [GO:0036440] (molecular function) Also known as: citrate (Re)-synthase activity, citrate (Si)-synthase activity, (R)-citrate synthase activity, (R)-citric synthase activity, Re-citrate-synthase activity, acetyl-CoA:oxaloacetate C-acetyltransferase [thioester-hydrolysing, (pro-R)-carboxymethyl-forming], acetyl-CoA:oxaloacetate C-acetyltransferase [thioester-hydrolysing, (pro-S)-carboxymethyl forming], citrate condensing enzyme activity, citrate oxaloacetate-lyase ((pro-3R)-CH(2)COO(-)->acetyl-CoA) activity, citrate oxaloacetate-lyase ((pro-3R)-CH2COO-rightacetyl-CoA), citrate oxaloacetate-lyase ((pro-3S)-CH(2)COO(-)->acetyl-CoA) activity, citrate oxaloacetate-lyase ((pro-3S)-CH2COO-rightacetyl-CoA), citrate oxaloacetate-lyase [(pro-3S)-CH2COOrightacetyl-CoA], citrate oxaloacetate-lyase, CoA-acetylating activity, citrate synthetase activity, citric synthase activity, citric-condensing enzyme activity, citrogenase activity, condensing enzyme activity, oxalacetic transacetase activity, oxaloacetate transacetase activity Relationships: is a type of GO:0046912 Definition: Catalysis of the reaction: acetyl-CoA + H2O + oxaloacetate = citrate + CoA. Sources: RHEA:16845